{
  "term_label": "mitochondrial membrane",
  "gene_name": "Cytochrome c oxidase subunit 7A-related protein, mitochondrial",
  "gene": "UniProtKB:O14548",
  "term_id": "GO:0031966",
  "gene_symbol": "COX7A2L"
}